{
  "gene": "UniProtKB:P56278",
  "gene_name": "Protein p13 MTCP-1",
  "term_label": "Unknown cellular component",
  "term_id": "UNKNOWN:0003",
  "gene_symbol": "MTCP1"
}